nitrile hydratase activity [GO:0018822] (molecular function) Relationships: is a type of hydro-lyase activity [GO:0016836] Sources: RHEA:12673 Definition: Catalysis of the reaction: an aliphatic amide = a nitrile + H2O. Subtypes: indole-3-acetonitrile nitrile hydratase activity [GO:0080109] Also known as: 3-cyanopyridine hydratase activity, H-NHase activity, L-NHase activity, NHase activity, acrylonitrile hydratase activity, aliphatic nitrile hydratase activity, aliphatic-amide hydro-lyase (nitrile-forming), nitrile hydro-lyase activity